{
  "gene": "UniProtKB:Q9ULC0",
  "gene_symbol": "EMCN",
  "gene_name": "Endomucin",
  "term_id": "UNKNOWN:0001",
  "term_label": "Unknown molecular function"
}